regulation of leukocyte adhesion to vascular endothelial cell [GO:1904994] (biological process) Subtypes: regulation of leukocyte tethering or rolling [GO:1903236], GO:1904995, positive regulation of leukocyte adhesion to vascular endothelial cell [GO:1904996], regulation of leukocyte adhesion to arterial endothelial cell [GO:1904997] Definition: Any process that modulates the frequency, rate or extent of leukocyte adhesion to vascular endothelial cell. Relationships: is_a GO:1903037; regulates leukocyte adhesion to vascular endothelial cell [GO:0061756] References: PMID:23897866 Sources: GOC:BHF, GOC:BHF_miRNA, GOC:TermGenie, GOC:bc, GO_REF:0000058